(2S,3R,6S,9S)-(-)-protoillud-7-ene synthase activity [GO:0061923] (molecular function) Also known as: protoillud-7-ene synthase activity References: PMID:27862766 Relationships: is a type of sesquiterpene synthase activity [GO:0010334] Definition: Catalysis of the reaction: 2-trans,6-trans-farnesyl diphosphate = diphosphate + (2S,3R,6S,9S)-(-)-protoillud-7-ene.